TFIIIC-class transcription factor complex binding [GO:0001156] (MF) Definition: Binding to a general RNA polymerase III transcription factor belonging to the TFIIC complex, one of the factors involved in formation of the preinitiation complex (PIC) by RNA polymerase III. References: PMID:12381659 Sources: GOC:txnOH Also known as: TFIIIC-class transcription factor binding Relationships: is a type of RNA polymerase III general transcription initiation factor binding [GO:0001025]